{
  "term_label": "plasma membrane",
  "gene": "UniProtKB:P35346",
  "gene_name": "Somatostatin receptor type 5",
  "gene_symbol": "SSTR5",
  "term_id": "GO:0005886"
}